{
  "gene_symbol": "ATN1",
  "term_label": "Unknown biological process",
  "gene_name": "Atrophin-1",
  "gene": "UniProtKB:P54259",
  "term_id": "UNKNOWN:0002"
}